cytoplasmic side of smooth endoplasmic reticulum membrane [GO:0098557] (cellular component) Definition: The side (leaflet) of the smooth endoplasmic reticulum membrane that faces the cytoplasm. Relationships: is_a GO:0098554; is part of GO:0030868 Sources: GOC:ab, GOC:dos